{
  "gene": "UniProtKB:Q8WXI8",
  "term_label": "antifungal innate immune response",
  "gene_name": "C-type lectin domain family 4 member D",
  "gene_symbol": "CLEC4D",
  "term_id": "GO:0061760"
}